{
  "term_label": "Unknown cellular component",
  "gene_name": "Zymogen granule membrane protein 16",
  "term_id": "UNKNOWN:0003",
  "gene": "UniProtKB:O60844",
  "gene_symbol": "ZG16"
}